{
  "gene_symbol": "USP43",
  "term_id": "UNKNOWN:0002",
  "gene": "UniProtKB:Q70EL4",
  "term_label": "Unknown biological process",
  "gene_name": "Ubiquitin carboxyl-terminal hydrolase 43"
}